{
  "term_label": "Unknown molecular function",
  "gene_symbol": "PODXL",
  "gene": "UniProtKB:O00592",
  "term_id": "UNKNOWN:0001",
  "gene_name": "Podocalyxin"
}